{
  "term_id": "GO:0000981",
  "gene_symbol": "GSX2",
  "gene": "UniProtKB:Q9BZM3",
  "term_label": "DNA-binding transcription factor activity, RNA polymerase II-specific",
  "gene_name": "GS homeobox 2"
}